positive regulation of response to external stimulus [GO:0032103] (biological process) Also known as: up regulation of response to external stimulus, up-regulation of response to external stimulus, upregulation of response to external stimulus, activation of response to external stimulus, stimulation of response to external stimulus Subtypes: positive regulation of antimicrobial humoral response [GO:0002760], positive regulation of lipopolysaccharide-mediated signaling pathway [GO:0031666], GO:0045089, positive regulation of axon regeneration [GO:0048680], positive regulation of inflammatory response [GO:0050729], positive regulation of chemotaxis [GO:0050921], negative regulation of fibrinolysis [GO:0051918], GO:0070961, positive regulation of defense response to insect [GO:1900367], positive regulation of defense response to bacterium [GO:1900426], positive regulation of systemic acquired resistance [GO:1901672], positive regulation of defense response to oomycetes [GO:1902290], positive regulation of chemokinesis [GO:1904367], GO:1904417, positive regulation of detection of mechanical stimulus involved in sensory perception of touch [GO:1905789], GO:1905792 Note: Note that this term is in the subset of terms that should not be used for direct gene product annotation. Instead, select a child term or, if no appropriate child term exists, please request a new term. Direct annotations to this term may be amended during annotation QC. Relationships: is_a regulation of response to external stimulus [GO:0032101]; is a type of positive regulation of response to stimulus [GO:0048584]; positively regulates response to external stimulus [GO:0009605] Definition: Any process that activates, maintains or increases the rate of a response to an external stimulus. Sources: GOC:mah